protein localization to mitotic spindle midzone [GO:1902967] (biological process) References: PMID:16824200 Sources: GOC:TermGenie, GO_REF:0000087 Also known as: protein localisation in mitotic spindle midzone, protein localisation to mitotic spindle midzone, protein localization in mitotic spindle midzone Relationships: is_a GO:1902480 Definition: A process in which a protein is transported to, or maintained in, a location within a mitotic spindle midzone.